{
  "gene": "UniProtKB:Q13136",
  "term_label": "synapse organization",
  "gene_symbol": "PPFIA1",
  "term_id": "GO:0050808",
  "gene_name": "Liprin-alpha-1"
}